{
  "gene": "UniProtKB:Q9BPX7",
  "gene_symbol": "C7orf25",
  "term_id": "UNKNOWN:0003",
  "gene_name": "UPF0415 protein C7orf25",
  "term_label": "Unknown cellular component"
}